{
  "gene_symbol": "CD207",
  "gene": "UniProtKB:Q9UJ71",
  "gene_name": "C-type lectin domain family 4 member K",
  "term_label": "carbohydrate binding",
  "term_id": "GO:0030246"
}